{
  "term_id": "GO:0038023",
  "gene_name": "Adiponectin receptor protein 2",
  "gene_symbol": "ADIPOR2",
  "term_label": "signaling receptor activity",
  "gene": "UniProtKB:Q86V24"
}